{
  "term_label": "Unknown biological process",
  "gene_name": "Small subunit processome component 20 homolog",
  "term_id": "UNKNOWN:0002",
  "gene": "UniProtKB:O75691",
  "gene_symbol": "UTP20"
}